{
  "gene_symbol": "CDC14C",
  "gene": "UniProtKB:A4D256",
  "term_id": "GO:0000226",
  "gene_name": "Dual specificity protein phosphatase CDC14C",
  "term_label": "microtubule cytoskeleton organization"
}